chromosome, centromeric core domain [GO:0034506] (cellular component) Relationships: is a type of GO:0098687; is part of GO:0000775 Definition: The innermost portion of the centromeric region of a chromosome, encompassing the core region of a chromosome centromere and the proteins that bind to it. Also known as: chromosome, centromeric core region, chromosome, centric core region Sources: GOC:mah, GOC:vw